{
  "term_label": "Ragulator complex",
  "gene": "UniProtKB:O43504",
  "gene_symbol": "LAMTOR5",
  "term_id": "GO:0071986",
  "gene_name": "Ragulator complex protein LAMTOR5"
}